regulation of Wnt signaling pathway, planar cell polarity pathway [GO:2000095] (biological process) Sources: GOC:BHF Subtypes: negative regulation of Wnt signaling pathway, planar cell polarity pathway [GO:0141113], positive regulation of Wnt signaling pathway, planar cell polarity pathway [GO:2000096] Definition: Any process that modulates the frequency, rate or extent of Wnt signaling pathway, planar cell polarity pathway. Relationships: is a type of GO:2000050; regulates Wnt signaling pathway, planar cell polarity pathway [GO:0060071] Also known as: regulation of PCP pathway, regulation of Wnt receptor signaling pathway, planar cell polarity pathway, regulation of Wnt receptor signalling pathway, planar cell polarity pathway, regulation of Wnt-activated signaling pathway, planar cell polarity pathway, regulation of Wnt-JNK signaling pathway, regulation of Wnt-PCP signaling pathway, regulation of non-canonical Wnt signaling pathway